{
  "term_label": "inner ear morphogenesis",
  "gene_symbol": "TMIE",
  "term_id": "GO:0042472",
  "gene": "UniProtKB:Q8NEW7",
  "gene_name": "Transmembrane inner ear expressed protein"
}